{
  "gene_symbol": "FLT3",
  "term_id": "GO:0004714",
  "term_label": "transmembrane receptor protein tyrosine kinase activity",
  "gene": "UniProtKB:P36888",
  "gene_name": "Receptor-type tyrosine-protein kinase FLT3"
}